{
  "term_id": "GO:0007266",
  "gene_name": "Tumor necrosis factor receptor superfamily member 16",
  "gene_symbol": "NGFR",
  "term_label": "Rho protein signal transduction",
  "gene": "UniProtKB:P08138"
}